{
  "gene_symbol": "MAP1LC3A",
  "gene_name": "Microtubule-associated proteins 1A_1B light chain 3A",
  "term_id": "GO:0000421",
  "gene": "UniProtKB:Q9H492",
  "term_label": "autophagosome membrane"
}